{
  "gene_name": "Uncharacterized protein C14orf93",
  "term_id": "UNKNOWN:0002",
  "gene": "UniProtKB:Q9H972",
  "term_label": "Unknown biological process",
  "gene_symbol": "C14orf93"
}